{
  "term_id": "GO:0061355",
  "gene_symbol": "PORCN",
  "gene_name": "Protein-serine O-palmitoleoyltransferase porcupine",
  "term_label": "Wnt protein secretion",
  "gene": "UniProtKB:Q9H237"
}